{
  "gene_name": "Adhesion G-protein coupled receptor F2",
  "gene": "UniProtKB:Q8IZF7",
  "term_label": "adenylate cyclase-activating G protein-coupled receptor signaling pathway",
  "gene_symbol": "ADGRF2P",
  "term_id": "GO:0007189"
}